{
  "term_id": "GO:0005654",
  "gene_symbol": "ZNF131",
  "gene_name": "Zinc finger protein 131",
  "term_label": "nucleoplasm",
  "gene": "UniProtKB:P52739"
}